{
  "gene": "UniProtKB:Q5VTR2",
  "gene_name": "E3 ubiquitin-protein ligase BRE1A",
  "term_label": "HULC complex",
  "gene_symbol": "RNF20",
  "term_id": "GO:0033503"
}